{
  "term_label": "Unknown molecular function",
  "gene": "UniProtKB:Q9Y678",
  "gene_name": "Coatomer subunit gamma-1",
  "gene_symbol": "COPG1",
  "term_id": "UNKNOWN:0001"
}